{
  "term_label": "Unknown cellular component",
  "term_id": "UNKNOWN:0003",
  "gene_symbol": "KLHL33",
  "gene": "UniProtKB:A6NCF5",
  "gene_name": "Kelch-like protein 33"
}